{
  "gene": "UniProtKB:Q5VWK0",
  "gene_symbol": "NBPF6",
  "term_id": "UNKNOWN:0002",
  "term_label": "Unknown biological process",
  "gene_name": "Neuroblastoma breakpoint family member 6"
}